L-glutamine biosynthetic process [GO:1901704] (biological process) Definition: The chemical reactions and pathways resulting in the formation of L-glutamine. Also known as: L-glutamine anabolism, L-glutamine biosynthesis, L-glutamine formation, L-glutamine synthesis Regulation: regulated by GO:0062132; negatively regulated by negative regulation of L-glutamine biosynthetic process [GO:0062133]; positively regulated by positive regulation of L-glutamine biosynthetic process [GO:0062134] Relationships: is a type of GO:0006542 Sources: GOC:TermGenie